{
  "gene_name": "Eukaryotic translation initiation factor 5B",
  "gene_symbol": "EIF5B",
  "gene": "UniProtKB:O60841",
  "term_id": "GO:0006413",
  "term_label": "translational initiation"
}